{
  "term_label": "sodium:bicarbonate symporter activity",
  "term_id": "GO:0008510",
  "gene_symbol": "SLC4A7",
  "gene": "UniProtKB:Q9Y6M7",
  "gene_name": "Sodium bicarbonate cotransporter 3"
}